{
  "gene_name": "[Pyruvate dehydrogenase [acetyl-transferring]]-phosphatase 1, mitochondrial",
  "gene_symbol": "PDP1",
  "term_id": "UNKNOWN:0002",
  "term_label": "Unknown biological process",
  "gene": "UniProtKB:Q9P0J1"
}